{
  "gene_symbol": "ALOX12",
  "gene_name": "Polyunsaturated fatty acid lipoxygenase ALOX12",
  "term_label": "lipoxygenase pathway",
  "term_id": "GO:0019372",
  "gene": "UniProtKB:P18054"
}